{
  "term_label": "diamine N-acetyltransferase activity",
  "term_id": "GO:0004145",
  "gene": "UniProtKB:P21673",
  "gene_name": "Diamine acetyltransferase 1",
  "gene_symbol": "SAT1"
}